{
  "gene_name": "Protein sel-1 homolog 2",
  "term_id": "GO:0005789",
  "term_label": "endoplasmic reticulum membrane",
  "gene": "UniProtKB:Q5TEA6",
  "gene_symbol": "SEL1L2"
}